{
  "term_label": "B cell receptor signaling pathway",
  "gene_name": "Tyrosine-protein kinase ITK_TSK",
  "gene_symbol": "ITK",
  "gene": "UniProtKB:Q08881",
  "term_id": "GO:0050853"
}